{
  "term_id": "GO:0009804",
  "gene_name": "Cytochrome P450 2A6",
  "term_label": "coumarin metabolic process",
  "gene": "UniProtKB:P11509",
  "gene_symbol": "CYP2A6"
}